{
  "gene_name": "FXYD domain-containing ion transport regulator 4",
  "gene": "UniProtKB:P59646",
  "gene_symbol": "FXYD4",
  "term_label": "sodium channel regulator activity",
  "term_id": "GO:0017080"
}